{
  "term_label": "RNA polymerase II cis-regulatory region sequence-specific DNA binding",
  "gene_name": "Homeobox protein MOX-2",
  "gene_symbol": "MEOX2",
  "term_id": "GO:0000978",
  "gene": "UniProtKB:P50222"
}